{
  "gene_symbol": "RELA",
  "gene": "UniProtKB:Q04206",
  "term_label": "inflammatory response",
  "term_id": "GO:0006954",
  "gene_name": "Transcription factor p65"
}